{
  "gene_symbol": "IMP3",
  "gene_name": "U3 small nucleolar ribonucleoprotein protein IMP3",
  "term_label": "rRNA processing",
  "gene": "UniProtKB:Q9NV31",
  "term_id": "GO:0006364"
}